{
  "gene_symbol": "OR8U1",
  "term_label": "Unknown molecular function",
  "gene_name": "Olfactory receptor 8U1",
  "term_id": "UNKNOWN:0001",
  "gene": "UniProtKB:Q8NH10"
}